aromatic amino acid family catabolic process to carboxylic acid via Ehrlich pathway [GO:0000952] (biological process) References: PMID:18281432 Sources: GOC:krc Definition: The chemical reactions and pathways involving the catabolism of amino acids to produce carboxylic acids with one carbon less than the starting amino acid. In S. cerevisiae, this is known to occur for leucine, isoleucine, valine, methionine, phenylalanine, tyrosine, or tryptophan. When an aromatic family amino acid, phenylalanine, tyrosine, or tryptophan, is used as the substrate, 2-phenylethanoate, 4-hydroxyphenylethanoate, or 2-(Indol-3-yl)-ethanoate, respectively, is produced. Often referred to as the Ehrlich pathway, these reactions generally occur during fermentation to produce a variety of carboxylic acids, sometimes collectively referred to as fusel acids. Depending on the redox state of the cells, alcohol derivatives may be produced instead of carboxylic acids. Relationships: is a type of amino acid catabolic process to carboxylic acid via Ehrlich pathway [GO:0000948]; is a type of aromatic amino acid family catabolic process [GO:0009074]